{
  "term_label": "isoprenoid biosynthetic process",
  "gene_name": "3-hydroxy-3-methylglutaryl-coenzyme A reductase",
  "gene_symbol": "HMGCR",
  "term_id": "GO:0008299",
  "gene": "UniProtKB:P04035"
}